peptidyl-cysteine oxidation [GO:0018171] (biological process) References: PMID:9586994 Sources: RESID:AA0205, RESID:AA0262 Relationships: is a type of protein oxidation [GO:0018158]; is a type of peptidyl-cysteine modification [GO:0018198] Definition: The oxidation of peptidyl-cysteine to peptidyl-L-cysteine sulfinic acid or peptidyl-L-cysteine sulfenic acid.